serotonin:sodium:chloride symporter activity [GO:0005335] (molecular function) Definition: Enables the transfer of a solute or solutes from one side of a membrane to the other according to the reaction: serotonin(out) + Na+(out) + Cl-(out) = serotonin(in) + Na+(in)+ Cl-(in). References: PMID:21752877, PMID:22519513 Relationships: is_a GO:0008504; is a type of sodium:chloride symporter activity [GO:0015378]; is part of GO:0051610 Also known as: serotonin transmembrane transporter activity, sodium/serotonin symporter activity, serotonin:sodium symporter activity